{
  "gene_name": "Carbohydrate sulfotransferase 10",
  "term_id": "GO:0030166",
  "gene_symbol": "CHST10",
  "gene": "UniProtKB:O43529",
  "term_label": "proteoglycan biosynthetic process"
}